{
  "gene_symbol": "RHEBL1",
  "gene_name": "GTPase RhebL1",
  "term_id": "GO:0005886",
  "gene": "UniProtKB:Q8TAI7",
  "term_label": "plasma membrane"
}